{
  "gene_name": "Zinc finger protein 74",
  "gene": "UniProtKB:Q16587",
  "term_id": "GO:0000978",
  "term_label": "RNA polymerase II cis-regulatory region sequence-specific DNA binding",
  "gene_symbol": "ZNF74"
}